{
  "term_id": "GO:0005085",
  "term_label": "guanyl-nucleotide exchange factor activity",
  "gene": "UniProtKB:Q8IV61",
  "gene_name": "Ras guanyl-releasing protein 3",
  "gene_symbol": "RASGRP3"
}